host cell lysosome [GO:0044187] (cellular component) Sources: GOC:jl Relationships: is a type of host intracellular membrane-bounded organelle [GO:0033648]; is_a host cell cytoplasm part [GO:0033655] Definition: A small lytic vacuole that has cell cycle-independent morphology and is found in most host animal cells and that contains a variety of hydrolases, most of which have their maximal activities in the pH range 5-6. The contained enzymes display latency if properly isolated. About 40 different lysosomal hydrolases are known and host cell lysosomes have a great variety of morphologies and functions.